starch utilization system complex assembly [GO:0044574] (biological process) Regulation: regulated by regulation of starch utilization system complex assembly [GO:1900512]; negatively regulated by GO:1900513; positively regulated by positive regulation of starch utilization system complex assembly [GO:1900514] Also known as: SUS complex assembly, assembly of starch utilization system complex Definition: The aggregation, arrangement and bonding together of the starch utilization system complex, a complex of cell envelope-associated proteins that degrades glycan. References: PMID:19553672, PMID:21219452 Sources: GOC:mengo_curators, GOC:tt Relationships: is a type of protein-containing complex assembly [GO:0065003]